{
  "gene_symbol": "MYPN",
  "gene_name": "Myopalladin",
  "gene": "UniProtKB:Q86TC9",
  "term_id": "GO:0030424",
  "term_label": "axon"
}